{
  "gene_name": "CKLF-like MARVEL transmembrane domain-containing protein 5",
  "gene": "UniProtKB:Q96DZ9",
  "gene_symbol": "CMTM5",
  "term_label": "Unknown molecular function",
  "term_id": "UNKNOWN:0001"
}